{
  "term_id": "GO:0003735",
  "gene_name": "Large ribosomal subunit protein bL27m",
  "gene_symbol": "MRPL27",
  "gene": "UniProtKB:Q9P0M9",
  "term_label": "structural constituent of ribosome"
}